negative regulation of centriole replication [GO:0046600] (biological process) Also known as: down regulation of centriole replication, down-regulation of centriole replication, downregulation of centriole replication, inhibition of centriole replication Definition: Any process that stops, prevents, or reduces the frequency, rate or extent of centriole replication. Sources: GOC:ai Relationships: is a type of negative regulation of centrosome duplication [GO:0010826]; is_a GO:0046599; is a type of negative regulation of organelle assembly [GO:1902116]; negatively regulates centriole replication [GO:0007099]